{
  "term_id": "GO:0008625",
  "term_label": "extrinsic apoptotic signaling pathway via death domain receptors",
  "gene_symbol": "CASP8AP2",
  "gene": "UniProtKB:Q9UKL3",
  "gene_name": "CASP8-associated protein 2"
}